{
  "term_id": "GO:0005730",
  "term_label": "nucleolus",
  "gene": "UniProtKB:Q6K0P9",
  "gene_symbol": "PYHIN1",
  "gene_name": "Pyrin and HIN domain-containing protein 1"
}